{
  "gene_name": "Rho GTPase-activating protein 23",
  "term_label": "Unknown biological process",
  "gene_symbol": "ARHGAP23",
  "gene": "UniProtKB:Q9P227",
  "term_id": "UNKNOWN:0002"
}